acetoin biosynthetic process [GO:0045151] (biological process) Definition: The chemical reactions and pathways resulting in the formation of acetoin, 3-hydroxy-2-butanone. Sources: GOC:mlg Also known as: acetoin anabolism, acetoin biosynthesis, acetoin formation, acetoin synthesis Relationships: is a type of ketone biosynthetic process [GO:0042181]; is a type of acetoin metabolic process [GO:0045149]; is a type of secondary alcohol biosynthetic process [GO:1902653]